{
  "term_label": "RNA polymerase II transcription regulatory region sequence-specific DNA binding",
  "gene_name": "Homeobox protein HMX1",
  "gene": "UniProtKB:Q9NP08",
  "term_id": "GO:0000977",
  "gene_symbol": "HMX1"
}